histamine binding [GO:0051381] (MF) Definition: Binding to histamine, a physiologically active amine, found in plant and animal tissue and released from mast cells as part of an allergic reaction in humans. Relationships: is a type of GO:0043169; is a type of heterocyclic compound binding [GO:1901363] Sources: GOC:ai